{
  "term_id": "GO:0003713",
  "gene_symbol": "SETD4",
  "gene": "UniProtKB:Q9NVD3",
  "gene_name": "SET domain-containing protein 4",
  "term_label": "transcription coactivator activity"
}